{
  "term_id": "GO:0006357",
  "term_label": "regulation of transcription by RNA polymerase II",
  "gene": "UniProtKB:Q8N7R0",
  "gene_symbol": "NANOGP1",
  "gene_name": "Putative homeobox protein NANOG2"
}